{
  "gene": "UniProtKB:Q9P055",
  "gene_symbol": "JKAMP",
  "gene_name": "JNK1_MAPK8-associated membrane protein",
  "term_id": "GO:0036503",
  "term_label": "ERAD pathway"
}